{
  "gene_symbol": "AATF",
  "gene_name": "Protein AATF",
  "gene": "UniProtKB:Q9NY61",
  "term_label": "Unknown biological process",
  "term_id": "UNKNOWN:0002"
}